{
  "gene": "UniProtKB:Q8IZ26",
  "term_id": "GO:0000981",
  "gene_symbol": "ZNF34",
  "gene_name": "Zinc finger protein 34",
  "term_label": "DNA-binding transcription factor activity, RNA polymerase II-specific"
}